{
  "term_id": "GO:0005886",
  "term_label": "plasma membrane",
  "gene": "UniProtKB:Q9GZP7",
  "gene_name": "Vomeronasal type-1 receptor 1",
  "gene_symbol": "VN1R1"
}